ANPR-A receptor complex [GO:1990620] (cellular component) Also known as: NPR1 receptor complex Definition: A receptor complex composed of two ANPR-A molecules and expressed in the heart atrium in mammals; it plays a major role in the regulation of blood pressure and salt-fluid volume homeostasis. Binding of the ligand AMP in response to atrial distension (high blood volume) leads to guanylate cyclase activity of the ANPR-A receptor complex, thereby elevating intracellular cGMP levels. The end result is a reduction in blood volume and, therefore, a reduction in cardiac output and systemic blood pressure. Note: An example of this is Npr1 in rat (UniProt symbol P18910) in PMID:15117952 (inferred from direct assay). References: PMID:15117952 Sources: GOC:ame Relationships: is a type of GO:0043235